{
  "gene_symbol": "FLCN",
  "gene": "UniProtKB:Q8NFG4",
  "gene_name": "Folliculin",
  "term_id": "GO:0000122",
  "term_label": "negative regulation of transcription by RNA polymerase II"
}